{
  "term_id": "UNKNOWN:0003",
  "gene_symbol": "EBF1",
  "gene_name": "Transcription factor COE1",
  "term_label": "Unknown cellular component",
  "gene": "UniProtKB:Q9UH73"
}